{
  "term_id": "GO:0043020",
  "term_label": "NADPH oxidase complex",
  "gene": "UniProtKB:Q86UR1",
  "gene_name": "NADPH oxidase activator 1",
  "gene_symbol": "NOXA1"
}